{
  "gene_name": "Tetratricopeptide repeat protein 7B",
  "gene_symbol": "TTC7B",
  "term_id": "GO:0072659",
  "gene": "UniProtKB:Q86TV6",
  "term_label": "protein localization to plasma membrane"
}